mannose biosynthetic process [GO:0019307] (biological process) Relationships: is_a mannose metabolic process [GO:0006013]; is a type of GO:0019319 Definition: The chemical reactions and pathways resulting in the formation of mannose, the aldohexose manno-hexose, the C-2 epimer of glucose. Also known as: mannose anabolism, mannose biosynthesis, mannose formation, mannose synthesis Sources: GOC:ai